{
  "term_id": "GO:0061630",
  "gene_name": "Nitric oxide synthase-interacting protein",
  "term_label": "ubiquitin protein ligase activity",
  "gene": "UniProtKB:Q9Y314",
  "gene_symbol": "NOSIP"
}